{
  "term_label": "negative regulation of transcription by RNA polymerase II",
  "term_id": "GO:0000122",
  "gene": "UniProtKB:Q9P0M6",
  "gene_name": "Core histone macro-H2A.2",
  "gene_symbol": "MACROH2A2"
}